alanine transmembrane transporter activity [GO:0022858] (molecular function) Subtypes: L-alanine transmembrane transporter activity [GO:0015180], alanine:sodium symporter activity [GO:0015655], D-alanine transmembrane transporter activity [GO:0042944], GO:0070906 Sources: GOC:mtg_transport, ISBN:0815340729 Relationships: is a type of neutral L-amino acid transmembrane transporter activity [GO:0015175]; is a type of GO:0046943; is part of alanine transport [GO:0032328] Definition: Enables the transfer of alanine from one side of a membrane to the other. Alanine is 2-aminopropanoic acid.